{
  "gene_name": "Heat shock transcription factor, X-linked member 3",
  "term_id": "GO:0000978",
  "gene": "UniProtKB:A0A1B0GWH4",
  "term_label": "RNA polymerase II cis-regulatory region sequence-specific DNA binding",
  "gene_symbol": "HSFX3"
}